vicianin beta-glucosidase activity [GO:0050392] (molecular function) Sources: EC:3.2.1.119, RHEA:14041 Definition: Catalysis of the reaction: (R)-vicianin + H2O = mandelonitrile + vicianose. Relationships: is a type of beta-glucosidase activity [GO:0008422] Also known as: vicianin b-glucosidase activity, (R)-vicianin beta-D-glucohydrolase activity, vicianin hydrolase activity